{
  "gene_name": "POU domain, class 4, transcription factor 3",
  "term_label": "DNA-binding transcription factor activity, RNA polymerase II-specific",
  "gene": "UniProtKB:Q15319",
  "gene_symbol": "POU4F3",
  "term_id": "GO:0000981"
}